{
  "term_id": "GO:0005777",
  "gene_symbol": "TYSND1",
  "gene": "UniProtKB:Q2T9J0",
  "gene_name": "Peroxisomal leader peptide-processing protease",
  "term_label": "peroxisome"
}